{
  "gene_symbol": "ZNF233",
  "gene": "UniProtKB:A6NK53",
  "term_id": "UNKNOWN:0003",
  "term_label": "Unknown cellular component",
  "gene_name": "Zinc finger protein 233"
}